{
  "gene_symbol": "SAA1",
  "term_id": "UNKNOWN:0001",
  "term_label": "Unknown molecular function",
  "gene": "UniProtKB:P0DJI8",
  "gene_name": "Serum amyloid A-1 protein"
}